{
  "gene_name": "Putative olfactory receptor 13C6",
  "term_label": "olfactory receptor activity",
  "term_id": "GO:0004984",
  "gene_symbol": "OR13C6P",
  "gene": "UniProtKB:Q8NH95"
}